{
  "gene_name": "C-C motif chemokine 25",
  "gene": "UniProtKB:O15444",
  "term_id": "GO:0070098",
  "term_label": "chemokine-mediated signaling pathway",
  "gene_symbol": "CCL25"
}